{
  "term_id": "GO:0004725",
  "gene_symbol": "PTPN9",
  "term_label": "protein tyrosine phosphatase activity",
  "gene_name": "Tyrosine-protein phosphatase non-receptor type 9",
  "gene": "UniProtKB:P43378"
}